ground meristem histogenesis [GO:0010066] (biological process) Definition: The formation of the primary meristem or meristematic tissue that gives rise to the ground tissues. Sources: GOC:tb, ISBN:0471245208 Relationships: is a type of primary meristem tissue development [GO:0010065]